{
  "gene_symbol": "GRIK4",
  "gene_name": "Glutamate receptor ionotropic, kainate 4",
  "term_label": "modulation of chemical synaptic transmission",
  "term_id": "GO:0050804",
  "gene": "UniProtKB:Q16099"
}